detoxification of sulfite [GO:0160245] (biological process) References: PMID:30859719 Definition: Any process that reduces or removes the toxicity of sulfite. These include transport of sulfite away from sensitive areas and to compartments or complexes whose purpose is sequestration of sulfite. Relationships: is a type of detoxification of inorganic compound [GO:0061687] Also known as: sulfite detoxification